{
  "gene_symbol": "NDRG4",
  "gene": "UniProtKB:Q9ULP0",
  "gene_name": "Protein NDRG4",
  "term_label": "signal transduction",
  "term_id": "GO:0007165"
}